{
  "term_label": "cupric reductase (NADH) activity",
  "gene": "UniProtKB:Q658P3",
  "gene_symbol": "STEAP3",
  "term_id": "GO:0008823",
  "gene_name": "Metalloreductase STEAP3"
}